{
  "gene": "UniProtKB:Q8N5Z5",
  "term_id": "GO:0031463",
  "term_label": "Cul3-RING ubiquitin ligase complex",
  "gene_symbol": "KCTD17",
  "gene_name": "BTB_POZ domain-containing protein KCTD17"
}